{
  "gene": "UniProtKB:Q9BY67",
  "gene_name": "Cell adhesion molecule 1",
  "term_id": "GO:0042271",
  "term_label": "susceptibility to natural killer cell mediated cytotoxicity",
  "gene_symbol": "CADM1"
}